Hpa2 acetyltransferase complex [GO:1990331] (cellular component) Relationships: is a type of H3 histone acetyltransferase complex [GO:0070775]; is a type of H4 histone acetyltransferase complex [GO:1902562] Definition: A tetrameric protein complex capable of acetyltransferase activity. It can catalyze the transfer of an acetyl group from acetyl-CoA to an acceptor residue on histone H-3, histone H-4, or on polyamines. The complex is also capable of acetylating certain small basic proteins. The two Hpa2 dimers that make up the tetramer are held together by interactions between the bound acetyl-CoA molecules. References: PMID:10600387 Sources: GOC:bhm